{
  "gene_symbol": "TRAJ44",
  "term_label": "Unknown biological process",
  "gene": "UniProtKB:A0A075B6X8",
  "gene_name": "T cell receptor alpha joining 44 (Fragment)",
  "term_id": "UNKNOWN:0002"
}